{
  "gene_name": "Beta-glucuronidase",
  "gene_symbol": "GUSB",
  "gene": "UniProtKB:P08236",
  "term_id": "GO:0030214",
  "term_label": "hyaluronan catabolic process"
}